{
  "gene": "UniProtKB:O75593",
  "gene_name": "Forkhead box protein H1",
  "term_id": "GO:0032444",
  "term_label": "activin responsive factor complex",
  "gene_symbol": "FOXH1"
}